{
  "gene_symbol": "CLDN3",
  "gene_name": "Claudin-3",
  "term_id": "GO:0007155",
  "term_label": "cell adhesion",
  "gene": "UniProtKB:O15551"
}